L-glutamine aminotransferase activity [GO:0070548] (molecular function) Definition: Catalysis of the transfer of an amino group from L-glutamine to an acceptor, usually a 2-oxo acid. Sources: GOC:mah Relationships: is a type of GO:0008483 Subtypes: glutamine-fructose-6-phosphate transaminase (isomerizing) activity [GO:0004360], glutamine-scyllo-inositol transaminase activity [GO:0047310], glutamine-phenylpyruvate transaminase activity [GO:0047316], L-glutamine:pyruvate aminotransferase activity [GO:0047945]